{
  "gene_name": "Cytochrome c oxidase assembly protein COX19",
  "term_label": "Unknown molecular function",
  "gene_symbol": "COX19",
  "gene": "UniProtKB:Q49B96",
  "term_id": "UNKNOWN:0001"
}